{
  "gene": "UniProtKB:P15531",
  "term_id": "GO:0004550",
  "gene_name": "Nucleoside diphosphate kinase A",
  "term_label": "nucleoside diphosphate kinase activity",
  "gene_symbol": "NME1"
}